{
  "gene_symbol": "SV2C",
  "term_id": "GO:0030672",
  "gene": "UniProtKB:Q496J9",
  "term_label": "synaptic vesicle membrane",
  "gene_name": "Synaptic vesicle glycoprotein 2C"
}